{
  "gene": "UniProtKB:Q68DV7",
  "term_label": "frizzled binding",
  "gene_name": "E3 ubiquitin-protein ligase RNF43",
  "gene_symbol": "RNF43",
  "term_id": "GO:0005109"
}